superoxide metabolic process [GO:0006801] (biological process) Subtypes: removal of superoxide radicals [GO:0019430], GO:0042554 Also known as: oxygen free radical metabolic process, oxygen free radical metabolism, superoxide free radical metabolic process, superoxide free radical metabolism, superoxide metabolism Definition: The chemical reactions and pathways involving superoxide, the superoxide anion O2- (superoxide free radical), or any compound containing this species. Relationships: is a type of reactive oxygen species metabolic process [GO:0072593] Regulation: regulated by regulation of superoxide metabolic process [GO:0090322] Sources: GOC:jl